response to toxic substance [GO:0009636] (biological process) Subtypes: response to herbicide [GO:0009635], response to mycotoxin [GO:0010046], response to microbial phytotoxin [GO:0010188], response to insecticide [GO:0017085], response to fungicide [GO:0060992], response to nematicide [GO:0093002], cellular response to toxic substance [GO:0097237] Also known as: detoxification response, toxin resistance, toxin susceptibility/resistance Definition: Any process that results in a change in state or activity of a cell or an organism (in terms of movement, secretion, enzyme production, gene expression, etc.) as a result of a toxic stimulus. Relationships: is a type of GO:0042221 Sources: GOC:lr